positive regulation of astrocyte differentiation [GO:0048711] (biological process) Also known as: up regulation of astrocyte differentiation, up-regulation of astrocyte differentiation, upregulation of astrocyte differentiation, activation of astrocyte differentiation, stimulation of astrocyte differentiation References: PMID:15139015 Sources: GOC:vp Definition: Any process that activates or increases the frequency, rate or extent of astrocyte differentiation. Relationships: is a type of GO:0045687; is_a regulation of astrocyte differentiation [GO:0048710]; positively regulates astrocyte differentiation [GO:0048708] Subtypes: GO:0061890